uracilylalanine synthase activity [GO:0050471] (molecular function) Relationships: is_a transferase activity, transferring alkyl or aryl (other than methyl) groups [GO:0016765] Sources: RHEA:11496 Definition: Catalysis of the reaction: O3-acetyl-L-serine + uracil = 3-(uracil-1-yl)-L-alanine + acetate. Also known as: 3-O-acetyl-L-serine:uracil 1-(2-amino-2-carboxyethyl)transferase activity, O(3)-acetyl-L-serine acetate-lyase (adding uracil) activity, O3-acetyl-L-serine acetate-lyase (adding uracil), O3-acetyl-L-serine:uracil 1-(2-amino-2-carboxyethyl)transferase activity, isowillardiine synthase activity, willardiine synthase activity